{
  "term_id": "GO:0005886",
  "gene_name": "Sodium_myo-inositol cotransporter 2",
  "term_label": "plasma membrane",
  "gene": "UniProtKB:Q8WWX8",
  "gene_symbol": "SLC5A11"
}